{
  "gene_name": "Cdc42 effector protein 4",
  "gene_symbol": "CDC42EP4",
  "term_label": "regulation of cell shape",
  "gene": "UniProtKB:Q9H3Q1",
  "term_id": "GO:0008360"
}